{
  "term_id": "GO:0006955",
  "gene_symbol": "IGLV5-45",
  "term_label": "immune response",
  "gene_name": "Immunoglobulin lambda variable 5-45",
  "gene": "UniProtKB:A0A087WSX0"
}